UTP binding [GO:0002134] (molecular function) Relationships: is a type of GO:0032557; is_a anion binding [GO:0043168] Definition: Binding to UTP, uridine 5'-triphosphate. Sources: GOC:hjd, ISBN:0198506732